{
  "gene_name": "POTE ankyrin domain family member B3",
  "term_label": "Unknown cellular component",
  "term_id": "UNKNOWN:0003",
  "gene_symbol": "POTEB3",
  "gene": "UniProtKB:A0JP26"
}